{
  "term_label": "Golgi apparatus",
  "gene": "UniProtKB:Q96G01",
  "gene_symbol": "BICD1",
  "term_id": "GO:0005794",
  "gene_name": "Protein bicaudal D homolog 1"
}